{
  "gene_name": "Synaptonemal complex central element protein 1",
  "gene_symbol": "SYCE1",
  "term_id": "UNKNOWN:0001",
  "gene": "UniProtKB:Q8N0S2",
  "term_label": "Unknown molecular function"
}